{
  "term_id": "GO:0045202",
  "gene_symbol": "HTR3A",
  "gene": "UniProtKB:P46098",
  "gene_name": "5-hydroxytryptamine receptor 3A",
  "term_label": "synapse"
}